negative regulation of embryo sac egg cell differentiation [GO:0045695] (biological process) Sources: GOC:go_curators, GOC:mtg_plant Relationships: is a type of negative regulation of cell differentiation [GO:0045596]; is a type of regulation of embryo sac egg cell differentiation [GO:0045694]; is a type of negative regulation of multicellular organismal process [GO:0051241]; is a type of GO:2000242; negatively regulates GO:0009560 Also known as: down regulation of female gametophyte egg cell differentiation, down-regulation of female gametophyte egg cell differentiation, downregulation of female gametophyte egg cell differentiation, negative regulation of female gametophyte egg cell differentiation, inhibition of female gametophyte egg cell differentiation Definition: Any process that stops, prevents, or reduces the frequency, rate or extent of embryo sac egg cell differentiation.